negative regulation of cold-induced thermogenesis [GO:0120163] (BP) Also known as: negative regulation of CIT Relationships: is a type of negative regulation of metabolic process [GO:0009892]; is a type of negative regulation of multicellular organismal process [GO:0051241]; is a type of regulation of cold-induced thermogenesis [GO:0120161]; negatively regulates cold-induced thermogenesis [GO:0106106] Definition: Any process that stops, prevents, or reduces the rate of cold-induced thermogenesis. References: PMID:27876809